positive regulation of osteoclast development [GO:2001206] (biological process) Definition: Any process that activates or increases the frequency, rate or extent of osteoclast development. Sources: GOC:obol Also known as: positive regulation of osteoclast cell development Relationships: is a type of positive regulation of osteoclast differentiation [GO:0045672]; is a type of GO:2001204; positively regulates osteoclast development [GO:0036035]